{
  "term_label": "plasma membrane",
  "gene_name": "Heat shock protein HSP 90-alpha",
  "gene_symbol": "HSP90AA1",
  "gene": "UniProtKB:P07900",
  "term_id": "GO:0005886"
}